{
  "gene_name": "C-C motif chemokine 7",
  "gene_symbol": "CCL7",
  "gene": "UniProtKB:P80098",
  "term_label": "chemokine-mediated signaling pathway",
  "term_id": "GO:0070098"
}